{
  "term_label": "cytoplasm",
  "gene_name": "Putative translationally-controlled tumor protein-like protein TPT1P8",
  "gene": "UniProtKB:Q9HAU6",
  "term_id": "GO:0005737",
  "gene_symbol": "TPT1P8"
}